{
  "gene": "UniProtKB:Q9BXA5",
  "term_label": "G protein-coupled receptor signaling pathway",
  "term_id": "GO:0007186",
  "gene_symbol": "SUCNR1",
  "gene_name": "Succinate receptor 1"
}